non-myelinated axon ensheathment in central nervous system [GO:0032293] (biological process) Definition: The process in which a non-myelinating glial cell membrane encircles an axon in the central nervous system. Sources: GOC:dgh Also known as: ensheathment of non-myelinated axons in central nervous system Relationships: is a type of GO:0032285; is a type of GO:0032291